{
  "term_label": "detection of chemical stimulus involved in sensory perception of smell",
  "gene_symbol": "OR2T12",
  "gene": "UniProtKB:Q8NG77",
  "gene_name": "Olfactory receptor 2T12",
  "term_id": "GO:0050911"
}